negative regulation of MAPK cascade [GO:0043409] (biological process) Subtypes: negative regulation of stress-activated MAPK cascade [GO:0032873], negative regulation of MAP kinase activity [GO:0043407], negative regulation of JNK cascade [GO:0046329], GO:0070373, negative regulation of ERK5 cascade [GO:0070377], negative regulation of pheromone response MAPK cascade [GO:0180040], GO:1903753 Relationships: is a type of regulation of MAPK cascade [GO:0043408]; is a type of negative regulation of intracellular signal transduction [GO:1902532]; negatively regulates GO:0000165 Also known as: down regulation of MAPK cascade, down regulation of MAPKKK cascade, down-regulation of MAPK cascade, down-regulation of MAPKKK cascade, downregulation of MAPK cascade, downregulation of MAPKKK cascade, negative regulation of MAP kinase cascade, negative regulation of MAP kinase kinase kinase cascade, negative regulation of MAPKKK cascade, negative regulation of mitogen activated protein kinase cascade, negative regulation of mitogen activated protein kinase kinase kinase cascade, negative regulation of mitogen-activated protein kinase cascade, negative regulation of mitogen-activated protein kinase kinase kinase cascade, inhibition of MAPK cascade, inhibition of MAPKKK cascade Definition: Any process that stops, prevents, or reduces the frequency, rate or extent of signal transduction mediated by the MAPKKK cascade. Sources: GOC:go_curators